DNA alkylation repair [GO:0006307] (biological process) Definition: The repair of alkylation damage in DNA, e.g. the removal of a non-physiological alkyl group from a nucleobase. This is usually mediated by DNA alkyltransferases. Also known as: DNA dealkylation involved in DNA repair References: PMID:10946226, PMID:35543797 Relationships: is_a DNA repair [GO:0006281]